positive regulation of peroxisome organization [GO:1900064] (biological process) References: PMID:7500953 Sources: GOC:TermGenie Also known as: positive regulation of peroxisome organisation, up regulation of peroxisome organisation, up-regulation of peroxisome organisation, upregulation of peroxisome organisation, activation of peroxisome organisation, activation of peroxisome organization, activation of peroxisome organization and biogenesis, activation of peroxisome-assembly ATPase activity, positive regulation of peroxisome organization and biogenesis, positive regulation of peroxisome-assembly ATPase activity, up regulation of peroxisome organization, up regulation of peroxisome organization and biogenesis, up regulation of peroxisome-assembly ATPase activity, up-regulation of peroxisome organization, up-regulation of peroxisome organization and biogenesis, up-regulation of peroxisome-assembly ATPase activity, upregulation of peroxisome organization, upregulation of peroxisome organization and biogenesis, upregulation of peroxisome-assembly ATPase activity Definition: Any process that activates or increases the frequency, rate or extent of peroxisome organization. Relationships: is a type of positive regulation of organelle organization [GO:0010638]; is a type of regulation of peroxisome organization [GO:1900063]; positively regulates peroxisome organization [GO:0007031]